{
  "term_id": "UNKNOWN:0002",
  "term_label": "Unknown biological process",
  "gene_name": "Protein NipSnap homolog 3B",
  "gene": "UniProtKB:Q9BS92",
  "gene_symbol": "NIPSNAP3B"
}